{
  "gene_symbol": "C7",
  "term_id": "GO:0006956",
  "gene_name": "Complement component C7",
  "gene": "UniProtKB:P10643",
  "term_label": "complement activation"
}